{
  "gene_name": "Dynein regulatory complex subunit 4",
  "term_id": "GO:0030317",
  "term_label": "flagellated sperm motility",
  "gene_symbol": "GAS8",
  "gene": "UniProtKB:O95995"
}